{
  "term_label": "magnesium ion transport",
  "gene": "UniProtKB:Q6NVV3",
  "term_id": "GO:0015693",
  "gene_symbol": "NIPAL1",
  "gene_name": "Magnesium transporter NIPA3"
}